negative regulation of induction of conjugation with cellular fusion [GO:0010515] (biological process) Definition: Any process that stops, prevents, or reduces the frequency or rate of initiation of conjugation with cellular fusion. Sources: GOC:dph, GOC:tb Relationships: is a type of negative regulation of conjugation with cellular fusion [GO:0031138]; RO_0002212 induction of conjugation with cellular fusion [GO:0010514]